{
  "gene": "UniProtKB:Q96P70",
  "gene_symbol": "IPO9",
  "gene_name": "Importin-9",
  "term_id": "GO:0005829",
  "term_label": "cytosol"
}